{
  "gene_name": "E3 ubiquitin-protein ligase COP1",
  "gene": "UniProtKB:Q8NHY2",
  "gene_symbol": "COP1",
  "term_label": "Unknown cellular component",
  "term_id": "UNKNOWN:0003"
}